{
  "term_id": "UNKNOWN:0003",
  "term_label": "Unknown cellular component",
  "gene_symbol": "SBSN",
  "gene": "UniProtKB:Q6UWP8",
  "gene_name": "Suprabasin"
}